{
  "gene_symbol": "ZSWIM3",
  "term_id": "UNKNOWN:0001",
  "gene_name": "Zinc finger SWIM domain-containing protein 3",
  "term_label": "Unknown molecular function",
  "gene": "UniProtKB:Q96MP5"
}